{
  "term_label": "protein O-linked glycosylation",
  "term_id": "GO:0006493",
  "gene_name": "Polypeptide N-acetylgalactosaminyltransferase 11",
  "gene_symbol": "GALNT11",
  "gene": "UniProtKB:Q8NCW6"
}